{
  "gene_name": "Zinc finger protein 567",
  "term_id": "UNKNOWN:0003",
  "term_label": "Unknown cellular component",
  "gene": "UniProtKB:Q8N184",
  "gene_symbol": "ZNF567"
}